{
  "gene_symbol": "MBD3L4",
  "gene": "UniProtKB:A6NDZ8",
  "term_label": "DNA methylation-dependent constitutive heterochromatin formation",
  "gene_name": "Putative methyl-CpG-binding domain protein 3-like 4",
  "term_id": "GO:0006346"
}